L-lactate dehydrogenase inhibitor activity [GO:0160193] (molecular function) Definition: Binds to and stops, prevents or reduces the activity of L-lactate dehydrogenase. References: PMID:33406399 Relationships: is a type of enzyme inhibitor activity [GO:0004857]; negatively regulates L-lactate dehydrogenase (NAD+) activity [GO:0004459]